{
  "gene_name": "AT-rich interactive domain-containing protein 4A",
  "term_label": "nucleus",
  "gene_symbol": "ARID4A",
  "term_id": "GO:0005634",
  "gene": "UniProtKB:P29374"
}